{
  "term_id": "GO:0000226",
  "gene_symbol": "TUBA3D",
  "term_label": "microtubule cytoskeleton organization",
  "gene": "UniProtKB:P0DPH8",
  "gene_name": "Tubulin alpha-3D chain"
}